{
  "gene_symbol": "AKAP3",
  "gene": "UniProtKB:O75969",
  "gene_name": "A-kinase anchor protein 3",
  "term_label": "cell surface receptor protein serine/threonine kinase signaling pathway",
  "term_id": "GO:0007178"
}